{
  "term_label": "plasma membrane",
  "gene_name": "Secreted Ly-6_uPAR domain-containing protein 2",
  "gene_symbol": "SLURP2",
  "term_id": "GO:0005886",
  "gene": "UniProtKB:P0DP57"
}